{
  "term_label": "Unknown molecular function",
  "gene_name": "COMM domain-containing protein 4",
  "gene_symbol": "COMMD4",
  "gene": "UniProtKB:Q9H0A8",
  "term_id": "UNKNOWN:0001"
}